{
  "gene_name": "Angiopoietin-related protein 5",
  "gene_symbol": "ANGPTL5",
  "gene": "UniProtKB:Q86XS5",
  "term_id": "UNKNOWN:0002",
  "term_label": "Unknown biological process"
}